{
  "gene_name": "Rapamycin-insensitive companion of mTOR",
  "gene": "UniProtKB:Q6R327",
  "gene_symbol": "RICTOR",
  "term_id": "GO:0038203",
  "term_label": "TORC2 signaling"
}